{
  "term_id": "GO:0030425",
  "gene_symbol": "KIF1B",
  "gene": "UniProtKB:O60333",
  "gene_name": "Kinesin-like protein KIF1B",
  "term_label": "dendrite"
}